{
  "gene": "UniProtKB:Q96G79",
  "gene_name": "Probable UDP-sugar transporter protein SLC35A4",
  "term_label": "transmembrane transporter activity",
  "gene_symbol": "SLC35A4",
  "term_id": "GO:0022857"
}